{
  "gene_symbol": "HEBP2",
  "term_id": "GO:0005737",
  "term_label": "cytoplasm",
  "gene_name": "Heme-binding protein 2",
  "gene": "UniProtKB:Q9Y5Z4"
}